{
  "term_label": "SNARE complex",
  "gene_symbol": "SNAP23",
  "term_id": "GO:0031201",
  "gene_name": "Synaptosomal-associated protein 23",
  "gene": "UniProtKB:O00161"
}